{
  "term_label": "plasma membrane",
  "gene": "UniProtKB:Q9NQS3",
  "term_id": "GO:0005886",
  "gene_symbol": "NECTIN3",
  "gene_name": "Nectin-3"
}